protein deglutamylation [GO:0035608] (biological process) Subtypes: C-terminal protein deglutamylation [GO:0035609], protein side chain deglutamylation [GO:0035610], GO:0035611 Relationships: is a type of peptidyl-glutamic acid modification [GO:0018200] Also known as: protein amino acid deglutamylation References: PMID:21074048 Sources: GOC:sp Definition: The removal of a glutamate residue from a protein. Glutamate residues in proteins can be gene-encoded, or added as side chains during the protein modification process of polyglutamylation.